{
  "term_label": "positive regulation of synapse assembly",
  "term_id": "GO:0051965",
  "gene": "UniProtKB:Q9NT99",
  "gene_symbol": "LRRC4B",
  "gene_name": "Leucine-rich repeat-containing protein 4B"
}